thiamine:proton symporter activity [GO:0034215] (molecular function) Definition: Enables the transfer of a solute or solutes from one side of a membrane to the other according to the reaction: thiamine(out) + H+(out) = thiamine(in) + H+(in). Sources: GOC:mah Also known as: thiamin:hydrogen symporter activity, thiamin:proton symporter activity, thiamine:hydrogen symporter activity Relationships: is a type of thiamine transmembrane transporter activity [GO:0015234]; is a type of GO:0015295 Subtypes: high-affinity thiamine:proton symporter activity [GO:0034216]